{
  "gene": "UniProtKB:Q8TCJ2",
  "term_label": "Unknown cellular component",
  "gene_name": "Dolichyl-diphosphooligosaccharide--protein glycosyltransferase subunit STT3B",
  "gene_symbol": "STT3B",
  "term_id": "UNKNOWN:0003"
}